{
  "gene_name": "Tubulin gamma-2 chain",
  "term_label": "gamma-tubulin ring complex",
  "gene": "UniProtKB:Q9NRH3",
  "term_id": "GO:0000931",
  "gene_symbol": "TUBG2"
}